{
  "gene_symbol": "SH3TC1",
  "term_label": "Unknown molecular function",
  "gene_name": "SH3 domain and tetratricopeptide repeat-containing protein 1",
  "gene": "UniProtKB:Q8TE82",
  "term_id": "UNKNOWN:0001"
}